mitochondrial histidyl-tRNA aminoacylation [GO:0070151] (biological process) Definition: The process of coupling histidine to histidyl-tRNA in a mitochondrion, catalyzed by histidyl-tRNA synthetase. In tRNA aminoacylation, the amino acid is first activated by linkage to AMP and then transferred to either the 2'- or the 3'-hydroxyl group of the 3'-adenosine residue of the tRNA. Relationships: is a type of histidyl-tRNA aminoacylation [GO:0006427]; is a type of tRNA aminoacylation for mitochondrial protein translation [GO:0070127] Sources: GOC:mah, GOC:mcc